{
  "gene_name": "Envoplakin",
  "gene": "UniProtKB:Q92817",
  "term_label": "structural molecule activity",
  "term_id": "GO:0005198",
  "gene_symbol": "EVPL"
}